{
  "term_id": "GO:0004984",
  "gene": "UniProtKB:Q8NGP4",
  "gene_name": "Olfactory receptor 5M3",
  "gene_symbol": "OR5M3",
  "term_label": "olfactory receptor activity"
}